uracil DNA N-glycosylase activity [GO:0004844] (molecular function) Relationships: is a type of deaminated base DNA N-glycosylase activity [GO:0097506] Subtypes: GO:0017065, G/U mismatch-specific uracil-DNA glycosylase activity [GO:0043739] References: PMID:9224623 Sources: GOC:elh, GOC:pr Also known as: uracil-DNA glycosylase activity Definition: Catalysis of the cleavage of the N-C1' glycosidic bond between the damaged DNA base and the deoxyribose sugar, releasing a free base and leaving an apyrimidinic (AP) site. Enzymes with this activity recognize and remove uracil bases in DNA that result from the deamination of cytosine or the misincorporation of dUTP opposite an adenine.